entry into diapause [GO:0055115] (BP) Sources: GOC:ds, GOC:jid, GOC:mah Relationships: is a type of dormancy process [GO:0022611] Definition: The dormancy process that results in entry into diapause. Diapause is a neurohormonally mediated, dynamic state of low metabolic activity. Associated characteristics of this form of dormancy include reduced morphogenesis, increased resistance to environmental extremes, and altered or reduced behavioral activity. Full expression develops in a species-specific manner, usually in response to a number of environmental stimuli that precede unfavorable conditions. Once diapause has begun, metabolic activity is suppressed even if conditions favorable for development prevail. Once initiated, only certain stimuli are capable of releasing the organism from this state, and this characteristic is essential in distinguishing diapause from hibernation. Subtypes: GO:0043053, GO:0055116